triterpenoid biosynthetic process [GO:0016104] (biological process) Definition: The chemical reactions and pathways resulting in the formation of triterpenoid compounds, terpenoids with six isoprene units. Subtypes: tricyclic triterpenoid biosynthetic process [GO:0010263], GO:0010686, pentacyclic triterpenoid biosynthetic process [GO:0019745], hopanoid biosynthetic process [GO:0019746] Sources: GOC:go_curators Relationships: is a type of GO:0006722; is_a terpenoid biosynthetic process [GO:0016114] Also known as: triterpenoid anabolism, triterpenoid biosynthesis, triterpenoid formation, triterpenoid synthesis, triterpene biosynthesis, triterpene biosynthetic process